{
  "term_label": "protein ubiquitination",
  "gene": "UniProtKB:Q15034",
  "term_id": "GO:0016567",
  "gene_symbol": "HERC3",
  "gene_name": "Probable E3 ubiquitin-protein ligase HERC3"
}